hindbrain formation [GO:0021576] (biological process) Sources: GOC:cls, GOC:dgh, GOC:dph, GOC:jid, GO_REF:0000021 Definition: The process that gives rise to the hindbrain. This process pertains to the initial formation of a structure from unspecified parts. The hindbrain is the region consisting of the medulla, pons and cerebellum. Areas of the hindbrain control motor and autonomic functions. Relationships: is a type of anatomical structure formation involved in morphogenesis [GO:0048646]; is part of GO:0021575